endoribonuclease complex [GO:1902555] (cellular component) Subtypes: ribonuclease MRP complex [GO:0000172], GO:0000214, ribonuclease P complex [GO:0030677], GO:0070578, Las1 complex [GO:0090730], bI4 intron splicing complex [GO:0106391], GO:0106392, GO:0120330, GO:0140638, ribonuclease III complex [GO:1903095], Ire1 complex [GO:1990332] References: PMID:18191223 Sources: GOC:TermGenie, GOC:bhm Definition: A protein complex which is capable of endoribonuclease activity. Relationships: is a type of endonuclease complex [GO:1905348]